{
  "gene": "UniProtKB:Q6L8H1",
  "gene_symbol": "KRTAP5-4",
  "term_id": "UNKNOWN:0002",
  "gene_name": "Keratin-associated protein 5-4",
  "term_label": "Unknown biological process"
}